{
  "term_id": "UNKNOWN:0001",
  "gene": "UniProtKB:Q96RN5",
  "gene_name": "Mediator of RNA polymerase II transcription subunit 15",
  "term_label": "Unknown molecular function",
  "gene_symbol": "MED15"
}